{
  "term_id": "GO:0010181",
  "term_label": "FMN binding",
  "gene_name": "Nitric oxide synthase 1",
  "gene_symbol": "NOS1",
  "gene": "UniProtKB:P29475"
}